4-oxoproline reductase activity [GO:0016617] (molecular function) Definition: Catalysis of the reaction: 4-hydroxy-L-proline + NAD+ = 4-oxoproline + NADH + H+. Sources: EC:1.1.1.104 Relationships: is_a oxidoreductase activity, acting on the CH-OH group of donors, NAD or NADP as acceptor [GO:0016616] Also known as: hydroxy-L-proline oxidase activity, 4-hydroxy-L-proline:NAD+ oxidoreductase activity, hydroxyproline oxidase activity